{
  "term_label": "nucleoplasm",
  "gene": "UniProtKB:Q92585",
  "gene_symbol": "MAML1",
  "gene_name": "Mastermind-like protein 1",
  "term_id": "GO:0005654"
}